{
  "term_label": "Unknown biological process",
  "gene_name": "Tyrosine-protein phosphatase non-receptor type 3",
  "gene": "UniProtKB:P26045",
  "gene_symbol": "PTPN3",
  "term_id": "UNKNOWN:0002"
}